{
  "term_label": "Unknown biological process",
  "gene_name": "Glutathione synthetase",
  "term_id": "UNKNOWN:0002",
  "gene": "UniProtKB:P48637",
  "gene_symbol": "GSS"
}